{
  "term_label": "Unknown molecular function",
  "gene": "UniProtKB:P20930",
  "gene_name": "Filaggrin",
  "gene_symbol": "FLG",
  "term_id": "UNKNOWN:0001"
}